{
  "gene": "UniProtKB:P21781",
  "term_label": "regulation of cell migration",
  "gene_symbol": "FGF7",
  "gene_name": "Fibroblast growth factor 7",
  "term_id": "GO:0030334"
}